{
  "term_id": "GO:0031410",
  "gene_name": "Occludin",
  "term_label": "cytoplasmic vesicle",
  "gene_symbol": "OCLN",
  "gene": "UniProtKB:Q16625"
}